{
  "gene": "UniProtKB:Q30KQ9",
  "term_id": "GO:0042056",
  "gene_symbol": "DEFB110",
  "gene_name": "Beta-defensin 110",
  "term_label": "chemoattractant activity"
}